{
  "term_label": "DNA-binding transcription factor activity, RNA polymerase II-specific",
  "term_id": "GO:0000981",
  "gene_name": "Zinc finger protein 468",
  "gene_symbol": "ZNF468",
  "gene": "UniProtKB:Q5VIY5"
}